hypochord development [GO:0055016] (biological process) Also known as: subnotochordal rod development Relationships: is a type of tissue development [GO:0009888]; is a type of embryonic organ development [GO:0048568] Definition: The process whose specific outcome is the progression of the hypochord over time, from its formation to the mature structure. The hypochord is a transient rod-like structure in the embryos of fish, lampreys and amphibians that is located immediately ventral to the notochord. The hypochord may play a role in positioning the dorsal aorta. Sources: GOC:devbiol, GOC:lb